{
  "term_id": "GO:0006003",
  "gene_symbol": "PFKFB2",
  "term_label": "fructose 2,6-bisphosphate metabolic process",
  "gene": "UniProtKB:O60825",
  "gene_name": "6-phosphofructo-2-kinase_fructose-2,6-bisphosphatase 2"
}